{
  "gene_name": "Ubiquitin-like-conjugating enzyme ATG10",
  "gene": "UniProtKB:Q9H0Y0",
  "gene_symbol": "ATG10",
  "term_label": "mitophagy",
  "term_id": "GO:0000423"
}